{
  "gene": "UniProtKB:Q9UBV2",
  "gene_name": "Protein sel-1 homolog 1",
  "term_label": "Unknown molecular function",
  "term_id": "UNKNOWN:0001",
  "gene_symbol": "SEL1L"
}